anterior region determination [GO:0007355] (biological process) Sources: ISBN:0879694238, http://fly.ebi.ac.uk/allied-data/lk/interactive-fly/aimain/1aahome.htm Relationships: is a type of GO:0009952; is part of zygotic determination of anterior/posterior axis, embryo [GO:0007354] Definition: Specification of the anterior (head and thoracic segments) of the embryo by the gap genes; exemplified in insects by the actions of hunchback gene product.